{
  "term_label": "Unknown biological process",
  "gene": "UniProtKB:Q96MF0",
  "gene_name": "Putative uncharacterized protein LOC100506887",
  "gene_symbol": "Q96MF0",
  "term_id": "UNKNOWN:0002"
}